{
  "gene": "UniProtKB:O00533",
  "gene_symbol": "CHL1",
  "gene_name": "Neural cell adhesion molecule L1-like protein",
  "term_id": "GO:0043005",
  "term_label": "neuron projection"
}